regulation of voltage-gated calcium channel activity [GO:1901385] (biological process) Relationships: is a type of regulation of transmembrane transporter activity [GO:0022898]; RO_0002211 voltage-gated calcium channel activity [GO:0005245] Subtypes: negative regulation of voltage-gated calcium channel activity [GO:1901386], GO:1901387 Definition: Any process that modulates the frequency, rate or extent of voltage-gated calcium channel activity. Also known as: regulation of depolarization-activated calcium channel, regulation of depolarization-activated voltage gated calcium channel activity, regulation of depolarization-activated voltage-gated calcium channel, regulation of depolarization-activated voltage-gated calcium channel activity, regulation of voltage gated calcium channel activity, regulation of voltage-dependent calcium channel activity, regulation of voltage-gated calcium ion channel activity, regulation of voltage-sensitive calcium channel, regulation of dihydropyridine-sensitive calcium channel activity Sources: GOC:BHF, GOC:TermGenie